{
  "gene_symbol": "RAB41",
  "gene": "UniProtKB:Q5JT25",
  "term_id": "GO:0003924",
  "term_label": "GTPase activity",
  "gene_name": "Ras-related protein Rab-41"
}